{
  "term_id": "GO:0031295",
  "gene": "UniProtKB:Q9NZQ7",
  "term_label": "T cell costimulation",
  "gene_name": "Programmed cell death 1 ligand 1",
  "gene_symbol": "CD274"
}